negative regulation of DNA-binding transcription factor activity [GO:0043433] (biological process) Sources: GOC:jl Relationships: is a type of negative regulation of molecular function [GO:0044092]; is a type of GO:0051090; negatively regulates DNA-binding transcription factor activity [GO:0003700] Also known as: negative regulation of transcription factor activity, down regulation of transcription factor activity, down-regulation of transcription factor activity, downregulation of transcription factor activity, negative regulation of DNA binding transcription factor activity, negative regulation of sequence-specific DNA binding transcription factor activity, inhibition of transcription factor activity, negative regulation of androgen receptor activity, negative regulation of thyroid hormone receptor activity Subtypes: negative regulation of NF-kappaB transcription factor activity [GO:0032088], GO:0032792 Definition: Any process that stops, prevents, or reduces the frequency, rate or extent of the activity of a transcription factor, any factor involved in the initiation or regulation of transcription.